{
  "term_id": "GO:0000922",
  "gene_symbol": "TPX2",
  "term_label": "spindle pole",
  "gene": "UniProtKB:Q9ULW0",
  "gene_name": "Targeting protein for Xklp2"
}